{
  "gene_name": "[Pyruvate dehydrogenase [acetyl-transferring]]-phosphatase 2, mitochondrial",
  "term_label": "Unknown biological process",
  "term_id": "UNKNOWN:0002",
  "gene": "UniProtKB:Q9P2J9",
  "gene_symbol": "PDP2"
}